{
  "gene_symbol": "MAPK14",
  "term_label": "cytoplasm",
  "gene_name": "Mitogen-activated protein kinase 14",
  "gene": "UniProtKB:Q16539",
  "term_id": "GO:0005737"
}